quinone catabolic process [GO:1901662] (biological process) Also known as: quinone breakdown, quinone catabolism, quinone degradation, quinone cofactor breakdown, quinone cofactor catabolic process, quinone cofactor catabolism, quinone cofactor degradation Sources: GOC:TermGenie, GOC:go_curators, GOC:pr Subtypes: ubiquinone catabolic process [GO:0032322] Definition: The chemical reactions and pathways resulting in the breakdown of quinone. Relationships: is a type of ketone catabolic process [GO:0042182]; is a type of quinone metabolic process [GO:1901661]